{
  "gene": "UniProtKB:Q9Y5J7",
  "term_id": "GO:0045039",
  "gene_name": "Mitochondrial import inner membrane translocase subunit Tim9",
  "term_label": "protein insertion into mitochondrial inner membrane",
  "gene_symbol": "TIMM9"
}